germarium-derived oocyte fate determination [GO:0007294] (biological process) Relationships: is a type of developmental process involved in reproduction [GO:0003006]; is a type of oocyte fate determination [GO:0030716]; is part of germarium-derived oocyte differentiation [GO:0030706] Sources: GOC:mtg_sensu, ISBN:0879694238 Also known as: maintenance of oocyte identity, oocyte cell fate determination Definition: The cell fate determination process in which a germarium-derived cell becomes capable of differentiating autonomously into an oocyte cell regardless of its environment; upon determination, the cell fate cannot be reversed. An example of this is found in Drosophila melanogaster.